{
  "term_label": "beta-alanine transmembrane transporter activity",
  "gene_name": "Sodium- and chloride-dependent neutral and basic amino acid transporter B(0+)",
  "term_id": "GO:0001761",
  "gene_symbol": "SLC6A14",
  "gene": "UniProtKB:Q9UN76"
}